phosphorylation-dependent protein binding [GO:0140031] (molecular function) Note: This term should only be used when the binding is shown to require phosphorylation of the target protein: the interaction needs to be tested with and without the PTM. The binding does not need to be at the site of phosphorylation. It may be that the phosphorylation causes a conformational change that allows binding of the protein to another region; this type of phosphorylation-dependent protein binding is valid for annotation to this term. Relationships: is a type of modification-dependent protein binding [GO:0140030] Definition: Binding to a protein upon phosphorylation of the target protein. References: PMID:26060076